{
  "gene_name": "Olfactory receptor",
  "gene_symbol": "OR5BS1",
  "term_label": "Unknown biological process",
  "term_id": "UNKNOWN:0002",
  "gene": "UniProtKB:A0A2R8YED5"
}